{
  "term_label": "CCR4-NOT complex",
  "gene_symbol": "CNOT11",
  "term_id": "GO:0030014",
  "gene": "UniProtKB:Q9UKZ1",
  "gene_name": "CCR4-NOT transcription complex subunit 11"
}